{
  "gene_symbol": "GYPB",
  "gene": "UniProtKB:P06028",
  "gene_name": "Glycophorin-B",
  "term_id": "UNKNOWN:0001",
  "term_label": "Unknown molecular function"
}